{
  "gene_symbol": "DYNC2H1",
  "term_id": "GO:0005930",
  "gene": "UniProtKB:Q8NCM8",
  "gene_name": "Cytoplasmic dynein 2 heavy chain 1",
  "term_label": "axoneme"
}